{
  "gene_symbol": "OR52K2",
  "term_label": "plasma membrane",
  "term_id": "GO:0005886",
  "gene_name": "Olfactory receptor 52K2",
  "gene": "UniProtKB:Q8NGK3"
}